preribosome binding [GO:1990275] (MF) References: PMID:22735702 Sources: GOC:di Relationships: is a type of GO:0043021 Definition: Binding to a preribosome.